{
  "term_label": "endocytic recycling",
  "gene_name": "Sorting nexin-7",
  "term_id": "GO:0032456",
  "gene_symbol": "SNX7",
  "gene": "UniProtKB:Q9UNH6"
}